{
  "term_label": "neurotransmitter receptor activity involved in regulation of postsynaptic cytosolic calcium ion concentration",
  "gene": "UniProtKB:Q13255",
  "gene_symbol": "GRM1",
  "gene_name": "Metabotropic glutamate receptor 1",
  "term_id": "GO:0099583"
}